{
  "gene_name": "Vam6_Vps39-like protein",
  "gene": "UniProtKB:Q96JC1",
  "term_id": "GO:0097352",
  "gene_symbol": "VPS39",
  "term_label": "autophagosome maturation"
}